methyl salicylate esterase activity [GO:0080031] (molecular function) Relationships: is a type of GO:0052689 References: PMID:18467465, PMID:18643994 Sources: RHEA:33611 Definition: Catalysis of the reaction: H2O + methyl salicylate = H+ + methanol + salicylate. Also known as: MESA esterase activity, methyl SA esterase activity, methylsalicylate esterase activity, salicylic acid methyl ester esterase activity